{
  "term_label": "acetylcholine receptor inhibitor activity",
  "gene_name": "Lymphocyte antigen 6E",
  "gene_symbol": "LY6E",
  "gene": "UniProtKB:Q16553",
  "term_id": "GO:0030550"
}